{
  "gene": "UniProtKB:P62857",
  "gene_name": "Small ribosomal subunit protein eS28",
  "term_label": "structural constituent of ribosome",
  "term_id": "GO:0003735",
  "gene_symbol": "RPS28"
}